{
  "term_label": "growth factor activity",
  "gene_name": "Fibroblast growth factor 1",
  "gene": "UniProtKB:P05230",
  "term_id": "GO:0008083",
  "gene_symbol": "FGF1"
}